seed germination [GO:0009845] (biological process) References: PMID:8281041 Relationships: is a type of multicellular organismal process [GO:0032501]; is part of GO:0090351 Subtypes: seed germination on parent plant [GO:0048623] Regulation: regulated by regulation of seed germination [GO:0010029]; positively regulated by positive regulation of seed germination [GO:0010030]; negatively regulated by negative regulation of seed germination [GO:0010187] Definition: The physiological and developmental changes that occur in a seed commencing with water uptake (imbibition) and terminating with the elongation of the embryonic axis.